{
  "term_id": "GO:0034599",
  "gene_symbol": "GPX8",
  "gene": "UniProtKB:Q8TED1",
  "term_label": "cellular response to oxidative stress",
  "gene_name": "Probable glutathione peroxidase 8"
}